type 7 metabotropic glutamate receptor binding [GO:0031804] (molecular function) Also known as: type 7 metabotropic glutamate receptor ligand Definition: Binding to a type 7 metabotropic glutamate receptor. Relationships: is a type of GO:0035256 Sources: GOC:mah, GOC:nln